quaternary ammonium group transport [GO:0015697] (biological process) Sources: GOC:ai, ISBN:0198506732 Also known as: quaternary amine transport, quaternary ammonium compound transport Definition: The directed movement into, out of or within a cell, or between cells, by means of some agent such as a transporter or pore of quaternary ammonium compounds, any compound that can be regarded as derived from ammonium hydroxide or an ammonium salt by replacement of all four hydrogen atoms of the NH4+ ion by organic groups. Subtypes: amino-acid betaine transport [GO:0015838], thiamine pyrophosphate transmembrane transport [GO:0030974], hydroxyectoine transmembrane transport [GO:0033308], GO:1902616, GO:2001143 Relationships: is_a nitrogen compound transport [GO:0071705]